{
  "gene_symbol": "NNAT",
  "gene": "UniProtKB:Q16517",
  "term_id": "UNKNOWN:0001",
  "term_label": "Unknown molecular function",
  "gene_name": "Neuronatin"
}